{
  "term_id": "UNKNOWN:0001",
  "gene_symbol": "BCAR1",
  "gene": "UniProtKB:P56945",
  "term_label": "Unknown molecular function",
  "gene_name": "Breast cancer anti-estrogen resistance protein 1"
}